{
  "term_label": "microtubule organizing center",
  "gene_symbol": "CLASP1",
  "gene": "UniProtKB:Q7Z460",
  "gene_name": "CLIP-associating protein 1",
  "term_id": "GO:0005815"
}